UTP diphosphatase activity [GO:0036221] (MF) References: PMID:17899088 Sources: GOC:dgf, RHEA:29395 Also known as: uridine triphosphate pyrophosphohydrolase activity Relationships: is a type of GO:0047429 Definition: Catalysis of the reaction: UTP + H2O = UMP + H+ + diphosphate.